response to nitrate starvation [GO:0090548] (biological process) Sources: GOC:tair_curators Relationships: is a type of response to starvation [GO:0042594] Definition: Any process that results in a change in state or activity of a cell or an organism (in terms of movement, secretion, enzyme production, gene expression, etc.) as a result of a starvation stimulus, deprivation of nitrate.